interleukin-16 receptor binding [GO:0045514] (molecular function) Relationships: is a type of GO:0005126 Definition: Binding to an interleukin-16 receptor. Sources: GOC:go_curators Also known as: IL-16, interleukin-16 receptor ligand